{
  "term_label": "apoptotic process",
  "gene_symbol": "DFFA",
  "gene": "UniProtKB:O00273",
  "gene_name": "DNA fragmentation factor subunit alpha",
  "term_id": "GO:0006915"
}